RasGAP-Fyn-Lyn-Yes complex [GO:0034996] (CC) Definition: A protein complex that consists of a GTPase activator protein (GAP) for Ras and three Src family protein tyrosine kinases, Fyn, Lyn and Yes. The complex is involved in signaling upon platelet activation. References: PMID:1544885 Also known as: p21(ras)GAP-Fyn-Lyn-Yes complex, thrombin stimulated Note: Note that the gene/protein name 'APC' should not be confused with the abbreviation for 'anaphase promoting complex'. Relationships: is a type of protein-containing complex [GO:0032991]; is part of cytoplasm [GO:0005737]